{
  "gene_symbol": "ARMCX2",
  "term_id": "GO:0005739",
  "gene": "UniProtKB:Q7L311",
  "gene_name": "Armadillo repeat-containing X-linked protein 2",
  "term_label": "mitochondrion"
}